negative regulation of amino acid metabolic process [GO:0045763] (biological process) Subtypes: negative regulation of arginine catabolic process [GO:1900082], negative regulation of tetrapyrrole biosynthetic process from glycine and succinyl-CoA [GO:1901414], negative regulation of gamma-aminobutyric acid catabolic process [GO:1901716], GO:1901997, negative regulation of ornithine catabolic process [GO:1903267], GO:1905013, negative regulation of glutamate metabolic process [GO:2000212], GO:2000283 Also known as: down regulation of amino acid metabolic process, down-regulation of amino acid metabolic process, downregulation of amino acid metabolic process, negative regulation of amino acid metabolism, inhibition of amino acid metabolic process Relationships: is a type of regulation of amino acid metabolic process [GO:0006521]; is a type of negative regulation of metabolic process [GO:0009892]; negatively regulates GO:0006520 Definition: Any process that stops, prevents, or reduces the frequency, rate or extent of the chemical reactions and pathways involving amino acid. Sources: GOC:go_curators